{
  "gene": "UniProtKB:Q6P597",
  "gene_symbol": "KLC3",
  "term_label": "microtubule-based movement",
  "term_id": "GO:0007018",
  "gene_name": "Kinesin light chain 3"
}